{
  "gene": "UniProtKB:A6NFN3",
  "term_label": "cytoplasm",
  "gene_name": "RNA binding protein fox-1 homolog 3",
  "term_id": "GO:0005737",
  "gene_symbol": "RBFOX3"
}